membrane-bounded organelle [GO:0043227] (cellular component) Relationships: is a type of GO:0043226; has part membrane [GO:0016020] Definition: Organized structure of distinctive morphology and function, bounded by a single or double lipid bilayer membrane. Includes the nucleus, mitochondria, plastids, vacuoles, and vesicles. Excludes the plasma membrane. Also known as: membrane-enclosed organelle Sources: GOC:go_curators Subtypes: cilium [GO:0005929], vesicle [GO:0031982], GO:0043231, extracellular membrane-bounded organelle [GO:0065010], spine apparatus [GO:0097444]